{
  "gene": "UniProtKB:P04085",
  "term_label": "angiogenesis",
  "term_id": "GO:0001525",
  "gene_symbol": "PDGFA",
  "gene_name": "Platelet-derived growth factor subunit A"
}